beta-catenin destruction complex [GO:0030877] (cellular component) Note: Note that the gene/protein name 'APC' should not be confused with the abbreviation for 'anaphase promoting complex'. Relationships: is a type of GO:0140535; is a type of catalytic complex [GO:1902494] References: PMID:14600025 Definition: A cytoplasmic protein complex containing glycogen synthase kinase-3-beta (GSK-3-beta), the adenomatous polyposis coli protein (APC), and the scaffolding protein axin, among others; phosphorylates beta-catenin, targets it for degradation by the proteasome. Also known as: APC-Axin-1-beta-catenin complex, Axin-APC-beta-catenin-GSK3B complex, BDC, beta-catenin degradation complex, 23S APC complex